{
  "gene_symbol": "C2orf73",
  "term_id": "UNKNOWN:0001",
  "term_label": "Unknown molecular function",
  "gene_name": "Uncharacterized protein C2orf73",
  "gene": "UniProtKB:Q8N5S3"
}